{
  "term_label": "Unknown cellular component",
  "term_id": "UNKNOWN:0003",
  "gene_symbol": "Q75L30",
  "gene_name": "Putative uncharacterized protein FLJ92257",
  "gene": "UniProtKB:Q75L30"
}